{
  "term_label": "cytoplasm",
  "gene_name": "Kelch repeat and BTB domain-containing protein 12",
  "gene": "UniProtKB:Q3ZCT8",
  "term_id": "GO:0005737",
  "gene_symbol": "KBTBD12"
}